{
  "gene_symbol": "MYT1L",
  "gene": "UniProtKB:Q9UL68",
  "term_id": "UNKNOWN:0001",
  "gene_name": "Myelin transcription factor 1-like protein",
  "term_label": "Unknown molecular function"
}